{
  "term_id": "UNKNOWN:0003",
  "gene_name": "Protein FAM131A",
  "gene_symbol": "FAM131A",
  "term_label": "Unknown cellular component",
  "gene": "UniProtKB:Q6UXB0"
}